orexin receptor activity [GO:0016499] (MF) Definition: Combining with orexin to initiate a change in cell activity. Relationships: is a type of G protein-coupled peptide receptor activity [GO:0008528] Sources: GOC:ai